negative regulation of presynaptic membrane organization [GO:1901630] (biological process) References: PMID:22426000 Sources: GOC:TermGenie Relationships: is a type of regulation of presynaptic membrane organization [GO:1901629]; is_a GO:1905809; negatively regulates presynaptic membrane organization [GO:0097090] Definition: Any process that stops, prevents or reduces the frequency, rate or extent of presynaptic membrane organization. Also known as: down regulation of presynaptic membrane organisation, down regulation of presynaptic membrane organization, down-regulation of presynaptic membrane organisation, down-regulation of presynaptic membrane organization, downregulation of presynaptic membrane organisation, downregulation of presynaptic membrane organization, negative regulation of pre-synaptic membrane organization, negative regulation of presynaptic membrane organisation, inhibition of presynaptic membrane organisation, inhibition of presynaptic membrane organization